mating projection tip membrane [GO:0070867] (cellular component) Sources: GOC:mah Definition: The portion of the plasma membrane surrounding a mating projection tip. Relationships: is a type of plasma membrane of cell tip [GO:0031520]; is part of mating projection tip [GO:0043332] Also known as: mating projection membrane fusion domain, shmoo tip membrane